response to very low light intensity stimulus [GO:0055122] (biological process) Subtypes: GO:0010203, cellular response to very low light intensity stimulus [GO:0071488] Relationships: is_a GO:0009642 Definition: Any process that results in a change in state or activity of a cell or an organism (in terms of movement, secretion, enzyme production, gene expression, etc.) as a result of a very low light intensity stimulus. A very low light intensity stimulus is defined as a level of electromagnetic radiation below 0.001 mmol/m2/sec. Sources: GOC:mtg_far_red